{
  "gene": "UniProtKB:Q15811",
  "term_label": "plasma membrane",
  "gene_symbol": "ITSN1",
  "gene_name": "Intersectin-1",
  "term_id": "GO:0005886"
}